melatonin receptor binding [GO:0031784] (molecular function) Definition: Binding to a melatonin receptor. Sources: GOC:mah, GOC:nln Also known as: melatonin receptor ligand Relationships: is a type of G protein-coupled receptor binding [GO:0001664] Subtypes: type 1A melatonin receptor binding [GO:0031785], type 1B melatonin receptor binding [GO:0031786], H9 melatonin receptor binding [GO:0031787]